signal transduction involved in cytokinesis checkpoint [GO:0072398] (biological process) Definition: A signal transduction process that contributes to a cytokinesis checkpoint. Sources: GOC:mtg_cell_cycle Relationships: is a type of mitotic cell cycle checkpoint signaling [GO:0007093]